{
  "gene_name": "Olfactory receptor 2A5",
  "gene": "UniProtKB:Q96R48",
  "term_id": "GO:0050911",
  "gene_symbol": "OR2A5",
  "term_label": "detection of chemical stimulus involved in sensory perception of smell"
}